negative regulation of border follicle cell migration [GO:1903687] (biological process) Relationships: is a type of negative regulation of epithelial cell migration [GO:0010633]; is a type of GO:1903684; negatively regulates border follicle cell migration [GO:0007298] Also known as: inhibition of border follicle cell migration References: PMID:18394891 Sources: GOC:TermGenie, GOC:als, GO_REF:0000058 Definition: Any process that stops, prevents or reduces the frequency, rate or extent of border follicle cell migration.